{
  "gene": "UniProtKB:Q5JU69",
  "term_label": "Unknown molecular function",
  "term_id": "UNKNOWN:0001",
  "gene_symbol": "TOR2A",
  "gene_name": "Torsin-2A"
}